{
  "term_id": "UNKNOWN:0002",
  "gene": "UniProtKB:P23142",
  "gene_name": "Fibulin-1",
  "term_label": "Unknown biological process",
  "gene_symbol": "FBLN1"
}